{
  "gene_name": "Eosinophil peroxidase",
  "gene": "UniProtKB:P11678",
  "term_id": "GO:0004601",
  "term_label": "peroxidase activity",
  "gene_symbol": "EPX"
}